{
  "gene_symbol": "GABRA1",
  "gene": "UniProtKB:P14867",
  "gene_name": "Gamma-aminobutyric acid receptor subunit alpha-1",
  "term_id": "GO:0022851",
  "term_label": "GABA-gated chloride ion channel activity"
}